{
  "gene_name": "Zinc finger protein 790",
  "term_label": "nucleus",
  "gene": "UniProtKB:Q6PG37",
  "gene_symbol": "ZNF790",
  "term_id": "GO:0005634"
}